{
  "gene_symbol": "MIA3",
  "gene_name": "Transport and Golgi organization protein 1 homolog",
  "term_label": "protein secretion",
  "gene": "UniProtKB:Q5JRA6",
  "term_id": "GO:0009306"
}